{
  "gene_symbol": "SLC17A1",
  "gene": "UniProtKB:Q14916",
  "term_label": "transmembrane transporter activity",
  "gene_name": "Sodium-dependent phosphate transport protein 1",
  "term_id": "GO:0022857"
}